glucose catabolic process [GO:0006007] (biological process) Subtypes: GO:0019595, glucose catabolic process to lactate [GO:0019659], GO:0030645, glucose catabolic process to pyruvate [GO:0061718] Definition: The chemical reactions and pathways resulting in the breakdown of glucose, the aldohexose gluco-hexose. Relationships: is a type of glucose metabolic process [GO:0006006]; is a type of hexose catabolic process [GO:0019320] Sources: GOC:ai Also known as: glucose breakdown, glucose catabolism, glucose degradation